{
  "term_label": "RNA polymerase II cis-regulatory region sequence-specific DNA binding",
  "gene_name": "Zinc finger and BTB domain-containing protein 7C",
  "gene_symbol": "ZBTB7C",
  "gene": "UniProtKB:A1YPR0",
  "term_id": "GO:0000978"
}